clustering of voltage-gated calcium channels [GO:0070073] (biological process) Also known as: clustering of voltage gated calcium channels, clustering of voltage-dependent calcium channels, voltage-gated calcium channel clustering Definition: The process in which voltage-gated calcium channels become localized together in high densities. References: PMID:18385325 Sources: GOC:BHF, GOC:sart Relationships: is a type of neuronal ion channel clustering [GO:0045161]